positive regulation of cholesterol storage [GO:0010886] (biological process) Sources: GOC:BHF, GOC:dph, GOC:tb Also known as: positive regulation of cholesterol sequestration Relationships: is a type of GO:0010884; is a type of regulation of cholesterol storage [GO:0010885]; positively regulates cholesterol storage [GO:0010878] Definition: Any process that increases the rate or extent of cholesterol storage. Cholesterol storage is the accumulation and maintenance in cells or tissues of cholesterol, cholest-5-en-3 beta-ol, the principal sterol of vertebrates and the precursor of many steroids, including bile acids and steroid hormones.